bulbus arteriosus formation [GO:0003234] (biological process) Definition: The developmental process pertaining to the initial formation of the bulbus arteriosus from unspecified parts. The bulbus arteriosus is an elastic chamber of the heart. Sources: GOC:mtg_heart Relationships: is a type of cardiac chamber formation [GO:0003207]; is part of GO:0003233